{
  "gene_symbol": "PRAMEF8",
  "term_label": "proteasome-mediated ubiquitin-dependent protein catabolic process",
  "gene": "UniProtKB:Q5VWM4",
  "gene_name": "PRAME family member 8",
  "term_id": "GO:0043161"
}